{
  "term_label": "nucleus",
  "gene": "UniProtKB:Q9UGU0",
  "gene_name": "Transcription factor 20",
  "gene_symbol": "TCF20",
  "term_id": "GO:0005634"
}